regulation of mitochondrial ATP synthesis coupled electron transport [GO:1905446] (biological process) Definition: Any process that modulates the frequency, rate or extent of mitochondrial ATP synthesis coupled electron transport. Relationships: is a type of regulation of generation of precursor metabolites and energy [GO:0043467]; regulates mitochondrial ATP synthesis coupled electron transport [GO:0042775] Subtypes: negative regulation of mitochondrial ATP synthesis coupled electron transport [GO:1905447], positive regulation of mitochondrial ATP synthesis coupled electron transport [GO:1905448] Also known as: regulation of mitochondrial electron transport, regulation of organelle ATP synthesis coupled electron transport References: PMID:23707074 Sources: GOC:PARL, GOC:TermGenie, GOC:bc, GO_REF:0000058